{
  "gene_name": "Interleukin-11 receptor subunit alpha",
  "term_id": "GO:0008284",
  "gene_symbol": "IL11RA",
  "gene": "UniProtKB:Q14626",
  "term_label": "positive regulation of cell population proliferation"
}